{
  "gene": "UniProtKB:Q96PR1",
  "term_label": "axon terminus",
  "gene_name": "Potassium voltage-gated channel subfamily C member 2",
  "gene_symbol": "KCNC2",
  "term_id": "GO:0043679"
}